{
  "term_label": "nucleus",
  "gene_symbol": "DUX4",
  "gene": "UniProtKB:Q9UBX2",
  "gene_name": "Double homeobox protein 4",
  "term_id": "GO:0005634"
}